{
  "gene_name": "Solute carrier family 35 member C2",
  "gene_symbol": "SLC35C2",
  "gene": "UniProtKB:Q9NQQ7",
  "term_id": "GO:0005793",
  "term_label": "endoplasmic reticulum-Golgi intermediate compartment"
}